protein formylation [GO:0018256] (biological process) Also known as: protein amino acid formylation Definition: The addition of a formyl group to a protein amino acid. Relationships: is a type of protein acylation [GO:0043543] Sources: GOC:ai Subtypes: N-terminal protein formylation [GO:0018004]